{
  "term_id": "GO:0005868",
  "gene": "UniProtKB:Q9Y6G9",
  "term_label": "cytoplasmic dynein complex",
  "gene_symbol": "DYNC1LI1",
  "gene_name": "Cytoplasmic dynein 1 light intermediate chain 1"
}